{
  "gene_name": "Arginine_serine-rich protein 1",
  "term_id": "UNKNOWN:0002",
  "term_label": "Unknown biological process",
  "gene_symbol": "RSRP1",
  "gene": "UniProtKB:Q9BUV0"
}